lipopolysaccharide catabolic process [GO:0009104] (biological process) Sources: GOC:ai Definition: The chemical reactions and pathways resulting in the breakdown of lipopolysaccharides, any of a group of related, structurally complex components of the outer membrane of Gram-negative bacteria. Also known as: LPS catabolic process, lipopolysaccharide breakdown, lipopolysaccharide catabolism, lipopolysaccharide degradation Relationships: is a type of lipopolysaccharide metabolic process [GO:0008653]; is_a GO:0009057; is a type of lipid catabolic process [GO:0016042]; is a type of carbohydrate derivative catabolic process [GO:1901136]